cellular response to lipid [GO:0071396] (biological process) Relationships: is_a response to lipid [GO:0033993]; is a type of cellular response to chemical stimulus [GO:0070887] Sources: GOC:mah Definition: Any process that results in a change in state or activity of a cell (in terms of movement, secretion, enzyme production, gene expression, etc.) as a result of a lipid stimulus. Subtypes: cellular response to sterol [GO:0036315], cellular response to abscisic acid stimulus [GO:0071215], cellular response to lipopolysaccharide [GO:0071222], GO:0071299, cellular response to retinoic acid [GO:0071300], cellular response to vitamin D [GO:0071305], cellular response to brassinosteroid stimulus [GO:0071367], cellular response to gibberellin stimulus [GO:0071370], cellular response to prostaglandin stimulus [GO:0071379], cellular response to steroid hormone stimulus [GO:0071383], cellular response to estradiol stimulus [GO:0071392], cellular response to testosterone stimulus [GO:0071394], GO:0071398, cellular response to triglyceride [GO:0071401], cellular response to lipid hydroperoxide [GO:0071449], GO:0072731, cellular response to farnesol [GO:0097308], GO:0106097, GO:1902348, cellular response to bile acid [GO:1903413], cellular response to dehydroepiandrosterone [GO:1903495], cellular response to micafungin [GO:1903968], cellular response to 2-O-acetyl-1-O-hexadecyl-sn-glycero-3-phosphocholine [GO:1904317], GO:1904322, cellular response to 1-oleoyl-sn-glycerol 3-phosphate [GO:1904566], cellular response to phorbol 13-acetate 12-myristate [GO:1904628], GO:1904630, GO:1905218, cellular response to borneol [GO:1905231], cellular response to beta-carotene [GO:1905388], cellular response to phosphatidylethanolamine [GO:1905712], cellular response to triterpenoid [GO:1905837]